background adaptation [GO:0120302] (biological process) Definition: Any process in which an organism changes its pigmentation (lightening in response to a brighter environment or darkening in response to a dimmer environment) in response to a change in light intensity. References: PMID:10493760, PMID:29239123, PMID:32898924 Sources: GOC:cvs, GOC:krc Relationships: is a type of GO:0009642; is a type of regulation of pigmentation [GO:0120305] Subtypes: GO:0120303, integument-mediated background adaptation [GO:0120304]